{
  "gene_symbol": "ZNF516",
  "gene": "UniProtKB:Q92618",
  "term_label": "DNA-binding transcription factor activity, RNA polymerase II-specific",
  "gene_name": "Zinc finger protein 516",
  "term_id": "GO:0000981"
}